{
  "term_label": "synaptic transmission, glutamatergic",
  "gene_symbol": "SLC17A6",
  "gene": "UniProtKB:Q9P2U8",
  "term_id": "GO:0035249",
  "gene_name": "Vesicular glutamate transporter 2"
}